{
  "term_label": "carbohydrate derivative binding",
  "gene_name": "Ficolin-1",
  "term_id": "GO:0097367",
  "gene_symbol": "FCN1",
  "gene": "UniProtKB:O00602"
}